{
  "term_id": "GO:0030154",
  "term_label": "cell differentiation",
  "gene_name": "ETS translocation variant 3",
  "gene": "UniProtKB:P41162",
  "gene_symbol": "ETV3"
}